{
  "gene_name": "Ras-related protein Rab-4A",
  "gene": "UniProtKB:P20338",
  "gene_symbol": "RAB4A",
  "term_label": "regulation of endocytosis",
  "term_id": "GO:0030100"
}